L-tryptophan conjugated cholate hydrolase activity [GO:7770009] (molecular function) Relationships: is a type of GO:7770003 References: PMID:40446798 Definition: Catalysis of the reaction: cholate + L-tryptophan = L-tryptophocholate + H2O.